exogenous lipid antigen binding [GO:0030884] (molecular function) References: PMID:14500461 Definition: Binding to an exogenous lipid antigen (examples include microbial lipids and glycolipids). Relationships: is a type of lipid antigen binding [GO:0030882]